{
  "gene_name": "RING finger protein 44",
  "gene_symbol": "RNF44",
  "term_id": "GO:0061630",
  "term_label": "ubiquitin protein ligase activity",
  "gene": "UniProtKB:Q7L0R7"
}